{
  "gene_symbol": "CDC42BPG",
  "term_label": "cytoskeleton",
  "term_id": "GO:0005856",
  "gene_name": "Serine_threonine-protein kinase MRCK gamma",
  "gene": "UniProtKB:Q6DT37"
}